{
  "term_label": "centriole",
  "gene": "UniProtKB:Q5U5Z8",
  "term_id": "GO:0005814",
  "gene_name": "Cytosolic carboxypeptidase 2",
  "gene_symbol": "AGBL2"
}